energy quenching [GO:1990066] (biological process) Definition: The process by which excess light energy absorbed by chlorophyll and not used to drive photosynthesis is emitted by nonphotochemical quenching or chlorophyll fluorescence. References: PMID:10938857 Relationships: is a type of response to light stimulus [GO:0009416] Subtypes: GO:0010196, GO:0090546